endospore core [GO:0070477] (cellular component) References: PMID:15035041, PMID:18035610 Sources: GOC:mah Definition: An intracellular part that represents the innermost portion of an endospore; the endospore core is dehydrated, enriched in dipicolinic acid and divalent cations, and metabolically inactive. Relationships: is a type of intracellular anatomical structure [GO:0005622]